lutein biosynthetic process [GO:0062171] (biological process) Definition: The chemical reactions and pathways resulting in the formation of lutein. References: PMID:24397433 Also known as: lutein anabolism, lutein biosynthesis, lutein formation Relationships: is a type of xanthophyll biosynthetic process [GO:0016123]